beta-agarase activity [GO:0033916] (molecular function) Definition: Catalysis of the hydrolysis of (1->4)-beta-D-galactosidic linkages in agarose, giving the tetramer as the predominant product. Also known as: agarase activity, agarose 3-glycanohydrolase activity, AgaA, AgaB, agarose 4-glycanohydrolase activity Sources: EC:3.2.1.81 Relationships: is a type of GO:0004553